{
  "gene_name": "N6-adenosine-methyltransferase non-catalytic subunit",
  "term_id": "GO:0016556",
  "gene_symbol": "METTL14",
  "term_label": "mRNA modification",
  "gene": "UniProtKB:Q9HCE5"
}